endocardial cushion to mesenchymal transition involved in heart valve formation [GO:0003199] (biological process) Also known as: endocardial cushion to mesenchymal transition involved in valve formation Relationships: is a type of endocardial cushion to mesenchymal transition [GO:0090500]; is part of heart valve formation [GO:0003188] Regulation: regulated by regulation of endocardial cushion to mesenchymal transition involved in heart valve formation [GO:2000800]; negatively regulated by negative regulation of endocardial cushion to mesenchymal transition involved in heart valve formation [GO:2000801]; positively regulated by GO:2000802 Definition: A transition where an endocardial cushion cell loses apical/basolateral polarity, severs intercellular adhesive junctions, degrades basement membrane components and becomes a migratory mesenchymal cell that will contribute to the formation of a cardiac valve. Sources: GOC:mtg_heart